ISG15-protein conjugation [GO:0032020] (biological process) Sources: GOC:mah Relationships: is a type of GO:0032446 Definition: The covalent addition to a protein of ISG15, a ubiquitin-like protein.